{
  "term_id": "UNKNOWN:0002",
  "gene_symbol": "GSN-AS1",
  "gene_name": "Putative uncharacterized protein GSN-AS1",
  "term_label": "Unknown biological process",
  "gene": "UniProtKB:Q9NRJ2"
}